progesterone biosynthetic process [GO:0006701] (biological process) Also known as: progesterone anabolism, progesterone biosynthesis, progesterone formation, progesterone synthesis Definition: The chemical reactions and pathways resulting in the formation of progesterone, a steroid hormone produced in the ovary which prepares and maintains the uterus for pregnancy. Also found in plants. Relationships: is a type of C21-steroid hormone biosynthetic process [GO:0006700]; is a type of GO:0042181; is a type of GO:0042448; is a type of olefinic compound biosynthetic process [GO:0120255] Regulation: regulated by regulation of progesterone biosynthetic process [GO:2000182]; negatively regulated by negative regulation of progesterone biosynthetic process [GO:2000183]; positively regulated by positive regulation of progesterone biosynthetic process [GO:2000184] References: PMID:14613534 Sources: GOC:jl